{
  "term_label": "protein deubiquitination involved in ubiquitin-dependent protein catabolic process",
  "gene_symbol": "ZRANB1",
  "term_id": "GO:0071947",
  "gene": "UniProtKB:Q9UGI0",
  "gene_name": "Ubiquitin thioesterase ZRANB1"
}